positive regulation of macropinocytosis [GO:1905303] (biological process) Definition: Any process that activates or increases the frequency, rate or extent of macropinocytosis. References: PMID:18691641 Sources: GOC:PARL, GOC:TermGenie, GOC:pad, GO_REF:0000058 Also known as: up regulation of macropinocytosis, up-regulation of macropinocytosis, upregulation of macropinocytosis, activation of macropinocytosis Relationships: is a type of GO:0048549; is_a regulation of macropinocytosis [GO:1905301]; positively regulates macropinocytosis [GO:0044351]